{
  "term_id": "UNKNOWN:0001",
  "gene_name": "Membrane-associated progesterone receptor component 2",
  "gene": "UniProtKB:O15173",
  "term_label": "Unknown molecular function",
  "gene_symbol": "PGRMC2"
}